{
  "term_id": "GO:0006414",
  "term_label": "translational elongation",
  "gene_name": "Elongation factor 1-alpha 1",
  "gene": "UniProtKB:P68104",
  "gene_symbol": "EEF1A1"
}